{
  "gene_name": "Metallothionein-1H",
  "term_id": "GO:0005737",
  "gene_symbol": "MT1H",
  "term_label": "cytoplasm",
  "gene": "UniProtKB:P80294"
}